{
  "gene_name": "Prolyl 4-hydroxylase subunit alpha-2",
  "term_id": "GO:0005783",
  "gene_symbol": "P4HA2",
  "gene": "UniProtKB:O15460",
  "term_label": "endoplasmic reticulum"
}